{
  "gene": "UniProtKB:P40394",
  "term_label": "all-trans-retinol dehydrogenase (NAD+) activity",
  "gene_symbol": "ADH7",
  "term_id": "GO:0004745",
  "gene_name": "All-trans-retinol dehydrogenase [NAD(+)] ADH7"
}